{
  "gene_symbol": "EXOSC3",
  "gene_name": "Exosome complex component RRP40",
  "gene": "UniProtKB:Q9NQT5",
  "term_label": "CUT catabolic process",
  "term_id": "GO:0071034"
}